{
  "gene_name": "CD276 antigen",
  "gene": "UniProtKB:Q5ZPR3",
  "term_label": "regulation of cytokine production",
  "term_id": "GO:0001817",
  "gene_symbol": "CD276"
}